ER-dependent peroxisome organization [GO:0032581] (BP) Definition: A process of peroxisome organization in which assembly or arrangement of constituent parts takes place in the endoplasmic reticulum. References: PMID:16717127, PMID:17646399 Sources: GOC:mah Relationships: is a type of GO:0007031 Also known as: ER-dependent peroxisome organisation, endoplasmic reticulum-dependent peroxisome organization, ER-dependent peroxisome biogenesis